{
  "term_label": "endocytosis",
  "gene_symbol": "RAB20",
  "gene": "UniProtKB:Q9NX57",
  "term_id": "GO:0006897",
  "gene_name": "Ras-related protein Rab-20"
}